{
  "gene_name": "RANBP2-like and GRIP domain-containing protein 2",
  "gene_symbol": "RGPD2",
  "gene": "UniProtKB:P0DJD1",
  "term_id": "GO:0005643",
  "term_label": "nuclear pore"
}